L-aminoadipate-semialdehyde dehydrogenase [NAD(P)+] activity [GO:0004043] (molecular function) Also known as: L-aminoadipate-semialdehyde dehydrogenase activity, 2-aminoadipate semialdehyde dehydrogenase activity, 2-aminoadipic semialdehyde dehydrogenase activity, AAR, L-2-aminoadipate-6-semialdehyde:NAD(P)+ 6-oxidoreductase, L-alpha-aminoadipate delta-semialdehyde oxidoreductase activity, L-alpha-aminoadipate delta-semialdehyde:NAD oxidoreductase activity, L-alpha-aminoadipate delta-semialdehyde:nicotinamide adenine dinucleotide oxidoreductase activity, alpha-aminoadipate reductase activity, alpha-aminoadipate-semialdehyde dehydrogenase activity, aminoadipate semialdehyde dehydrogenase activity, aminoadipate-semialdehyde dehydrogenase activity Relationships: is a type of aldehyde dehydrogenase [NAD(P)+] activity [GO:0004030] Sources: EC:1.2.1.31 Definition: Catalysis of the reaction: (S)-2-amino-6-oxohexanoate + NAD(P)+ + H2O = L-2-aminoadipate + NAD(P)H + 2 H+.